cellular response to decane [GO:1902783] (biological process) Relationships: is a type of cellular response to alkane [GO:1902779]; is a type of response to decane [GO:1902782] References: PMID:23826995 Sources: GOC:TermGenie, GOC:mengo_curators, GO_REF:0000071 Definition: Any process that results in a change in state or activity of a cell (in terms of movement, secretion, enzyme production, gene expression, etc.) as a result of a decane stimulus.